{
  "term_label": "estrogen metabolic process",
  "gene_symbol": "UGT2B7",
  "term_id": "GO:0008210",
  "gene": "UniProtKB:P16662",
  "gene_name": "UDP-glucuronosyltransferase 2B7"
}